{
  "term_label": "axoneme",
  "gene_name": "Phosphatidylinositol polyphosphate 5-phosphatase type IV",
  "gene_symbol": "INPP5E",
  "term_id": "GO:0005930",
  "gene": "UniProtKB:Q9NRR6"
}